8-hydroxy-5-deazaflavin:NADPH oxidoreductase activity [GO:0102261] (molecular function) Definition: Catalysis of the reaction: NADP+ + reduced coenzyme F420-(gamma-L-Glu)(n) = 2 H+ + NADPH + oxidized coenzyme F420-(gamma-L-Glu)(n). Relationships: is a type of oxidoreductase activity, acting on the CH-NH group of donors, NAD or NADP as acceptor [GO:0016646] Also known as: F420-dependent NADP reductase activity References: PMID:11726492 Sources: RHEA:31363